wide pore channel activity [GO:0022829] (molecular function) Subtypes: GO:0005243, GO:0015288, GO:0055077 Definition: Enables the energy-independent facilitated diffusion of propanediol through a large pore, un-gated channel. Examples include gap junctions, which transport substances from one cell to another; and porins which transport substances in and out of bacteria, mitochondria and chloroplasts. Also known as: non-gated, wide pore channel activity, gap junction activity Sources: GOC:mtg_transport, ISBN:0815340729 Relationships: is a type of channel activity [GO:0015267]